{
  "term_label": "plasma membrane",
  "term_id": "GO:0005886",
  "gene": "UniProtKB:Q9BT40",
  "gene_name": "Inositol polyphosphate 5-phosphatase K",
  "gene_symbol": "INPP5K"
}